lipoarabinomannan binding [GO:0001876] (MF) References: PMID:10586073 Relationships: is a type of GPI anchor binding [GO:0034235] Definition: Binding to lipoarabinomannan. Also known as: LAM binding